{
  "term_id": "GO:0120192",
  "gene_name": "Multiple PDZ domain protein",
  "gene_symbol": "MPDZ",
  "gene": "UniProtKB:O75970",
  "term_label": "tight junction assembly"
}